{
  "term_id": "GO:0005385",
  "term_label": "zinc ion transmembrane transporter activity",
  "gene": "UniProtKB:Q6P5W5",
  "gene_symbol": "SLC39A4",
  "gene_name": "Zinc transporter ZIP4"
}